{
  "gene": "UniProtKB:Q7Z6B7",
  "gene_name": "SLIT-ROBO Rho GTPase-activating protein 1",
  "term_id": "GO:0005096",
  "gene_symbol": "SRGAP1",
  "term_label": "GTPase activator activity"
}